cardiac chamber morphogenesis [GO:0003206] (biological process) Sources: GOC:mtg_heart Definition: The process in which a cardiac chamber is generated and organized. A cardiac chamber is an enclosed cavity within the heart. Regulation: regulated by regulation of cardiac chamber morphogenesis [GO:1901219]; negatively regulated by GO:1901220; positively regulated by positive regulation of cardiac chamber morphogenesis [GO:1901221] Also known as: heart chamber morphogenesis Relationships: is a type of anatomical structure morphogenesis [GO:0009653]; is part of GO:0003007; is part of GO:0003205 Subtypes: cardiac ventricle morphogenesis [GO:0003208], GO:0003209, bulbus arteriosus morphogenesis [GO:0003233], sinus venosus morphogenesis [GO:0003236], GO:0003239